{
  "gene": "UniProtKB:P30279",
  "term_id": "GO:0005815",
  "gene_symbol": "CCND2",
  "term_label": "microtubule organizing center",
  "gene_name": "G1_S-specific cyclin-D2"
}